{
  "term_label": "mitotic actomyosin contractile ring assembly actin filament organization",
  "gene": "UniProtKB:Q13576",
  "term_id": "GO:1903479",
  "gene_name": "Ras GTPase-activating-like protein IQGAP2",
  "gene_symbol": "IQGAP2"
}